{
  "gene": "UniProtKB:Q8WYN0",
  "term_label": "cysteine-type endopeptidase activity",
  "term_id": "GO:0004197",
  "gene_symbol": "ATG4A",
  "gene_name": "Cysteine protease ATG4A"
}